{
  "gene_symbol": "HLA-H",
  "gene": "UniProtKB:P01893",
  "term_id": "GO:0002476",
  "term_label": "antigen processing and presentation of endogenous peptide antigen via MHC class Ib",
  "gene_name": "Putative HLA class I histocompatibility antigen, alpha chain H"
}